{
  "term_label": "establishment of mitotic spindle orientation",
  "gene_name": "F-box_WD repeat-containing protein 11",
  "term_id": "GO:0000132",
  "gene_symbol": "FBXW11",
  "gene": "UniProtKB:Q9UKB1"
}